{
  "gene": "UniProtKB:Q8N0Z9",
  "term_label": "cell-cell adhesion",
  "term_id": "GO:0098609",
  "gene_symbol": "VSIG10",
  "gene_name": "V-set and immunoglobulin domain-containing protein 10"
}